{
  "gene_symbol": "EIF4A2",
  "term_label": "cytoplasmic translational initiation",
  "gene": "UniProtKB:Q14240",
  "gene_name": "Eukaryotic initiation factor 4A-II",
  "term_id": "GO:0002183"
}